{
  "gene_symbol": "LSM14B",
  "gene": "UniProtKB:Q9BX40",
  "term_label": "mRNA binding",
  "gene_name": "Protein LSM14 homolog B",
  "term_id": "GO:0003729"
}